{
  "gene": "UniProtKB:P22570",
  "gene_symbol": "FDXR",
  "term_label": "ferredoxin-NADP+ reductase activity",
  "term_id": "GO:0004324",
  "gene_name": "NADPH:adrenodoxin oxidoreductase, mitochondrial"
}